{
  "term_id": "UNKNOWN:0001",
  "gene_name": "Phosphatidylinositol N-acetylglucosaminyltransferase subunit P",
  "term_label": "Unknown molecular function",
  "gene": "UniProtKB:P57054",
  "gene_symbol": "PIGP"
}